{
  "term_id": "GO:0006955",
  "gene_name": "Immunoglobulin kappa variable 1-5",
  "term_label": "immune response",
  "gene": "UniProtKB:P01602",
  "gene_symbol": "IGKV1-5"
}